{
  "term_label": "Golgi cisterna membrane",
  "gene_name": "Golgin subfamily A member 6C",
  "gene": "UniProtKB:A6NDK9",
  "gene_symbol": "GOLGA6C",
  "term_id": "GO:0032580"
}